{
  "gene_name": "Leucine-rich repeat LGI family member 4",
  "gene": "UniProtKB:Q8N135",
  "term_label": "neuron maturation",
  "term_id": "GO:0042551",
  "gene_symbol": "LGI4"
}